{
  "term_label": "mitochondrial matrix",
  "gene": "UniProtKB:Q8N1Q8",
  "gene_name": "Acyl-coenzyme A thioesterase THEM5",
  "gene_symbol": "THEM5",
  "term_id": "GO:0005759"
}